{
  "gene": "UniProtKB:Q9NVE4",
  "term_label": "Unknown cellular component",
  "gene_symbol": "CCDC87",
  "gene_name": "Coiled-coil domain-containing protein 87",
  "term_id": "UNKNOWN:0003"
}